{
  "gene": "UniProtKB:Q07812",
  "gene_symbol": "BAX",
  "term_label": "intrinsic apoptotic signaling pathway in response to DNA damage",
  "term_id": "GO:0008630",
  "gene_name": "Apoptosis regulator BAX"
}